{
  "term_label": "cytoplasm",
  "gene_symbol": "SULT1C3",
  "term_id": "GO:0005737",
  "gene": "UniProtKB:Q6IMI6",
  "gene_name": "Sulfotransferase 1C3"
}